{
  "term_label": "heme binding",
  "term_id": "GO:0020037",
  "gene_symbol": "HBQ1",
  "gene": "UniProtKB:P09105",
  "gene_name": "Hemoglobin subunit theta-1"
}